{
  "gene_name": "Interleukin-6",
  "term_label": "cytokine activity",
  "gene": "UniProtKB:P05231",
  "term_id": "GO:0005125",
  "gene_symbol": "IL6"
}